{
  "gene_name": "Ras-GEF domain-containing family member 1C",
  "term_id": "GO:0005085",
  "gene_symbol": "RASGEF1C",
  "term_label": "guanyl-nucleotide exchange factor activity",
  "gene": "UniProtKB:Q8N431"
}